mycolate cell wall layer assembly [GO:0071769] (biological process) Also known as: mycolate cell wall layer biogenesis Relationships: is a type of GO:0022607; is part of Actinobacterium-type cell wall biogenesis [GO:0071766] Definition: The aggregation, arrangement and bonding together of a set of components, including arabinogalactan mycolate and trehalose dimycolate, to form the mycolate layer of the Actinobacterium-type cell wall. The mycolate layer is physically attached to the peptidoglycan layer. References: PMID:15653820, PMID:3149973 Sources: GOC:mah, MetaCyc:PWY-6397